{
  "gene": "UniProtKB:P30531",
  "term_id": "GO:0035725",
  "gene_name": "Sodium- and chloride-dependent GABA transporter 1",
  "term_label": "sodium ion transmembrane transport",
  "gene_symbol": "SLC6A1"
}